symbiont-mediated perturbation of host erythrocyte aggregation [GO:0020013] (biological process) Definition: Any process in which a symbiont organism modulates the frequency, rate or extent of erythrocyte aggregation in its host organism, e.g. the binding of parasite-infected erythrocytes to uninfected erythrocytes. Relationships: is a type of GO:0044068 References: PMID:19467172, PMID:21305024 Sources: GOC:add, GOC:dgh, GOC:mb, GOC:pr Note: Please note that this term does not refer to the in vitro assay called erythrocyte rosetting. Also known as: modulation by symbiont of host erythrocyte aggregation, rosetting